{
  "term_label": "regulation of small GTPase mediated signal transduction",
  "gene": "UniProtKB:Q9P2N2",
  "gene_symbol": "ARHGAP28",
  "term_id": "GO:0051056",
  "gene_name": "Rho GTPase-activating protein 28"
}